negative regulation of miRNA-mediated gene silencing [GO:0060965] (biological process) Definition: A process that decreases the rate, frequency, or extent of gene silencing by a microRNA (miRNA). Subtypes: target-directed miRNA degradation [GO:0140958], GO:1903799 Also known as: negative regulation of gene silencing by miRNA, negative regulation of gene silencing by microRNA Relationships: is a type of GO:0060964; is a type of negative regulation of post-transcriptional gene silencing by regulatory ncRNA [GO:1900369]; RO_0002212 miRNA-mediated post-transcriptional gene silencing [GO:0035195] References: PMID:23985560, PMID:28379604 Sources: GOC:aruk, GOC:bc, GOC:dph, GOC:rl, GOC:tb